{
  "term_label": "lipoprotein lipase activity",
  "gene_symbol": "PNLIPRP2",
  "gene": "UniProtKB:P54317",
  "gene_name": "Pancreatic lipase-related protein 2",
  "term_id": "GO:0004465"
}